regulation of chaperone-mediated protein complex assembly [GO:0090034] (biological process) Subtypes: positive regulation of chaperone-mediated protein complex assembly [GO:0090035] Sources: GOC:BHF, GOC:dph, GOC:tb Definition: Any process that modulates the frequency, rate, or extent of chaperone-mediated protein complex assembly. Chaperone-mediated protein complex assembly is the aggregation, arrangement and bonding together of a set of components to form a protein complex, mediated by chaperone molecules that do not form part of the finished complex. Relationships: is a type of regulation of protein-containing complex assembly [GO:0043254]; regulates chaperone-mediated protein complex assembly [GO:0051131]